{
  "gene": "UniProtKB:A6NDX5",
  "gene_name": "Putative zinc finger protein 840",
  "term_id": "GO:0005634",
  "term_label": "nucleus",
  "gene_symbol": "ZNF840P"
}